Lsm-containing SMN-Sm protein complex [GO:0034731] (cellular component) Relationships: is a type of GO:0034719 References: PMID:12975319, PMID:17401408 Also known as: SMN-containing protein complex Definition: An SMN-Sm protein complex formed by the association of the methylated Sm proteins B/B', D3, E, F, and G, and Lsm10 and Lsm11, with the SMN complex. This complex forms Sm cores on U7 snRNA.